origin recognition complex assembly [GO:1902561] (biological process) Also known as: ORC assembly, ORC formation, origin of replication recognition complex assembly, origin of replication recognition complex formation, origin recognition complex formation Definition: The aggregation, arrangement and bonding together of a set of components to form an origin recognition complex. Relationships: is a type of protein-containing complex assembly [GO:0065003] References: PMID:11717425 Sources: GOC:TermGenie